cellooligosaccharide binding [GO:2001064] (MF) Definition: Binding to cellooligosaccharide. Relationships: is a type of oligosaccharide binding [GO:0070492] Sources: GOC:mengo_curators